{
  "term_id": "GO:0003007",
  "gene_name": "Mesoderm posterior protein 1",
  "gene": "UniProtKB:Q9BRJ9",
  "gene_symbol": "MESP1",
  "term_label": "heart morphogenesis"
}